{
  "gene_symbol": "SELENOP",
  "term_id": "GO:0005576",
  "gene_name": "Selenoprotein P",
  "term_label": "extracellular region",
  "gene": "UniProtKB:P49908"
}